MHC class I protein binding, via antigen binding groove [GO:0023027] (molecular function) Relationships: is a type of MHC class I protein binding [GO:0042288]; is part of MHC class I protein complex binding [GO:0023024] Definition: Binding to a major histocompatibility complex class I molecules via the antigen binding groove. Sources: GOC:mtg_signal, GOC:vw